{
  "gene_name": "Kinesin-like protein KIF22",
  "gene": "UniProtKB:Q14807",
  "term_id": "GO:0005737",
  "term_label": "cytoplasm",
  "gene_symbol": "KIF22"
}